{
  "gene": "UniProtKB:Q7Z3J3",
  "term_label": "nuclear pore",
  "gene_name": "RanBP2-like and GRIP domain-containing protein 4",
  "gene_symbol": "RGPD4",
  "term_id": "GO:0005643"
}